{
  "gene_symbol": "CD2AP",
  "gene": "UniProtKB:Q9Y5K6",
  "term_label": "protein-macromolecule adaptor activity",
  "gene_name": "CD2-associated protein",
  "term_id": "GO:0030674"
}